{
  "gene_symbol": "MPP7",
  "term_id": "GO:0005886",
  "term_label": "plasma membrane",
  "gene_name": "MAGUK p55 subfamily member 7",
  "gene": "UniProtKB:Q5T2T1"
}